{
  "gene_name": "ATPase family AAA domain-containing protein 2",
  "gene_symbol": "ATAD2",
  "term_label": "transcription initiation-coupled chromatin remodeling",
  "term_id": "GO:0045815",
  "gene": "UniProtKB:Q6PL18"
}